{
  "term_label": "eukaryotic translation initiation factor 4F complex",
  "gene": "UniProtKB:Q04637",
  "gene_symbol": "EIF4G1",
  "gene_name": "Eukaryotic translation initiation factor 4 gamma 1",
  "term_id": "GO:0016281"
}